{
  "term_label": "Unknown biological process",
  "gene": "UniProtKB:Q9BXE9",
  "term_id": "UNKNOWN:0002",
  "gene_name": "Vomeronasal type-1 receptor 3",
  "gene_symbol": "VN1R3"
}